ABC-type D-xylose transporter activity [GO:0015614] (molecular function) Sources: RHEA:29899 Relationships: is a type of D-xylose transmembrane transporter activity [GO:0015148]; is_a ABC-type monosaccharide transporter activity [GO:0015407] Definition: Enables the transfer of a solute or solutes from one side of a membrane to the other according to the reaction: ATP + H2O + D-xylose(out) = ADP + phosphate + D-xylose(in). Also known as: D-xylose porter activity, ATPase-coupled D-xylose transmembrane transporter activity, D-xylose-importing ATPase activity